{
  "gene_name": "Upstream stimulatory factor 2",
  "gene": "UniProtKB:Q15853",
  "term_label": "regulation of transcription by RNA polymerase II",
  "term_id": "GO:0006357",
  "gene_symbol": "USF2"
}